azurophil granule [GO:0042582] (cellular component) References: PMID:17152095, PMID:28717070, PMID:5914694 Sources: GOC:jl, WIKIPEDIA:Azurophilic_granule Relationships: is a type of primary lysosome [GO:0005766]; is a type of GO:0030141 Also known as: primary granule Definition: Primary lysosomal granule readily stainable with a Romanowsky stain.